{
  "gene": "UniProtKB:Q5U623",
  "term_label": "regulation of DNA-templated transcription",
  "gene_name": "Activating transcription factor 7-interacting protein 2",
  "term_id": "GO:0006355",
  "gene_symbol": "ATF7IP2"
}